negative regulation of amide metabolic process [GO:0034249] (biological process) Also known as: negative regulation of amide metabolism, negative regulation of cellular amide metabolic process Relationships: is a type of GO:0009892; is a type of GO:0034248; negatively regulates amide metabolic process [GO:0043603] Definition: Any process that stops, prevents, or reduces the frequency, rate or extent of the chemical reactions and pathways involving amides. Sources: GOC:mah Subtypes: negative regulation of penicillin catabolic process [GO:0033248], negative regulation of amide catabolic process [GO:0034252], negative regulation of peptide hormone processing [GO:0060570], negative regulation of pyruvate decarboxylation to acetyl-CoA [GO:0160218], negative regulation of ceramide biosynthetic process [GO:1900060], negative regulation of penicillin biosynthetic process [GO:1900197], GO:1900495, negative regulation of butyryl-CoA catabolic process to butanol [GO:1900498], negative regulation of butyryl-CoA catabolic process to butyrate [GO:1900501], negative regulation of emericellamide biosynthetic process [GO:1900659], negative regulation of gliotoxin biosynthetic process [GO:1900690], negative regulation of tensidol A biosynthetic process [GO:1900708], negative regulation of tensidol B biosynthetic process [GO:1900711], negative regulation of pseurotin A biosynthetic process [GO:1900850], GO:1901414, negative regulation of amyloid-beta formation [GO:1902430], negative regulation of glutathione biosynthetic process [GO:1903787], negative regulation of ferrichrome biosynthetic process [GO:1905569], negative regulation of isopentenyl diphosphate biosynthetic process, mevalonate pathway [GO:2001211]